{
  "gene_symbol": "ICE2",
  "gene": "UniProtKB:Q659A1",
  "term_id": "GO:0042796",
  "gene_name": "Little elongation complex subunit 2",
  "term_label": "snRNA transcription by RNA polymerase III"
}